photosystem II [GO:0009523] (cellular component) Relationships: is a type of photosystem [GO:0009521] Definition: A photosystem that contains a pheophytin-quinone reaction center with associated accessory pigments and electron carriers. In cyanobacteria and chloroplasts, in the presence of light, PSII functions as a water-plastoquinone oxidoreductase, transferring electrons from water to plastoquinone, whereas other photosynthetic bacteria carry out anoxygenic photosynthesis and oxidize other compounds to re-reduce the photoreaction center. References: PMID:9821949 Sources: GOC:ds, GOC:mah, ISBN:0943088399 Subtypes: chloroplast photosystem II [GO:0030095], GO:0030096